{
  "gene_name": "Testis-specific Y-encoded-like protein 5",
  "gene_symbol": "TSPYL5",
  "term_id": "GO:0003682",
  "gene": "UniProtKB:Q86VY4",
  "term_label": "chromatin binding"
}